regulation of intrinsic apoptotic signaling pathway in response to hydrogen peroxide [GO:1903750] (biological process) Also known as: regulation of hydrogen peroxide-induced apoptosis, regulation of hydrogen peroxide-induced intrinsic apoptotic signaling pathway, regulation of intrinsic apoptotic signaling pathway in response to H2O2, regulation of H2O2-induced intrinsic apoptotic signaling pathway Relationships: is a type of regulation of hydrogen peroxide-mediated programmed cell death [GO:1901298]; is a type of regulation of oxidative stress-induced intrinsic apoptotic signaling pathway [GO:1902175]; RO_0002211 GO:0036481 References: PMID:18681888 Sources: GOC:TermGenie, GO_REF:0000058 Subtypes: regulation of hydrogen peroxide-induced neuron intrinsic apoptotic signaling pathway [GO:1903383], GO:1903751, GO:1903752 Definition: Any process that modulates the frequency, rate or extent of intrinsic apoptotic signaling pathway in response to hydrogen peroxide.